adenosylcobinamide kinase activity [GO:0043752] (molecular function) Definition: Catalysis of the reaction: RTP + adenosylcobinamide = adenosylcobinamide phosphate + RDP (where RTP is either ATP or GTP). Also known as: AdoCbi kinase/AdoCbi-phosphate guanylyltransferase, adenosylcobinamide kinase/adenosylcobinamide-phosphate guanylyltransferase, RTP:adenosylcobinamide phosphotransferase activity, cobinamide kinase activity, adenosylcobinamide kinase (ATP-specific) activity, adenosylcobinamide kinase (GTP-specific) activity, CobU Sources: EC:2.7.1.156 Relationships: is a type of GO:0016301; is a type of phosphotransferase activity, alcohol group as acceptor [GO:0016773]